{
  "gene_symbol": "GAK",
  "gene_name": "Cyclin-G-associated kinase",
  "gene": "UniProtKB:O14976",
  "term_label": "clathrin-dependent endocytosis",
  "term_id": "GO:0072583"
}